interleukin-17A production [GO:0097087] (biological process) Also known as: IL-17A production, interleukin-17A biosynthetic process Regulation: regulated by regulation of interleukin-17A production [GO:0150151]; negatively regulated by negative regulation of interleukin-17A production [GO:0150152]; positively regulated by positive regulation of interleukin-17A production [GO:0150153] Relationships: is a type of interleukin-17 production [GO:0032620] References: PMID:27901018 Sources: GOC:rv Definition: The appearance of interleukin-17A due to biosynthesis or secretion following a cellular stimulus, resulting in an increase in its intracellular or extracellular levels.